{
  "gene": "UniProtKB:Q6F5E8",
  "gene_symbol": "CARMIL2",
  "term_label": "regulation of Arp2/3 complex-mediated actin nucleation",
  "term_id": "GO:0034315",
  "gene_name": "Capping protein, Arp2_3 and myosin-I linker protein 2"
}